{
  "gene_name": "Nuclear factor of activated T-cells, cytoplasmic 1",
  "term_label": "transcription regulator complex",
  "term_id": "GO:0005667",
  "gene": "UniProtKB:O95644",
  "gene_symbol": "NFATC1"
}